positive regulation of RNA polymerase II transcription preinitiation complex assembly [GO:0045899] (biological process) Also known as: positive regulation of RNA polymerase II transcriptional pre-initiation complex assembly, positive regulation of RNA polymerase II transcriptional pre-initiation complex biosynthesis, positive regulation of RNA polymerase II transcriptional preinitiation complex assembly, positive regulation of RNA polymerase II transcriptional preinitiation complex formation, up regulation of RNA polymerase II transcriptional preinitiation complex assembly, up-regulation of RNA polymerase II transcriptional preinitiation complex assembly, upregulation of RNA polymerase II transcriptional preinitiation complex assembly, activation of RNA polymerase II transcriptional preinitiation complex assembly, stimulation of RNA polymerase II transcriptional preinitiation complex assembly Sources: GOC:go_curators Relationships: is a type of positive regulation of protein-containing complex assembly [GO:0031334]; is a type of regulation of RNA polymerase II transcription preinitiation complex assembly [GO:0045898]; is a type of GO:0060261; positively regulates RNA polymerase II preinitiation complex assembly [GO:0051123] Definition: Any process that activates or increases the frequency, rate or extent of RNA polymerase II transcriptional preinitiation complex assembly.